{
  "gene": "UniProtKB:Q8N5M1",
  "term_label": "Unknown molecular function",
  "gene_name": "ATP synthase mitochondrial F1 complex assembly factor 2",
  "term_id": "UNKNOWN:0001",
  "gene_symbol": "ATPAF2"
}